{
  "term_id": "GO:0005886",
  "term_label": "plasma membrane",
  "gene_symbol": "PLPP2",
  "gene": "UniProtKB:O43688",
  "gene_name": "Phospholipid phosphatase 2"
}